{
  "gene_symbol": "PEG10",
  "term_label": "mRNA binding",
  "term_id": "GO:0003729",
  "gene": "UniProtKB:Q86TG7",
  "gene_name": "Retrotransposon-derived protein PEG10"
}